{
  "gene_name": "Transcriptional regulator Kaiso",
  "gene": "UniProtKB:Q86T24",
  "gene_symbol": "ZBTB33",
  "term_label": "nucleoplasm",
  "term_id": "GO:0005654"
}